viral capsid, major subunit [GO:0098017] (CC) Definition: The part of the viral capsid that comprises the most common capsomere type. For example, in a T=3 icosahedral capsid, which is composed of 12 pentameric and 20 hexameric capsomeres, the hexameric capsomeres are major subunits. Relationships: is a type of capsomere [GO:0046727] Also known as: major capsomere, major head protein Sources: GOC:bm